negative regulation of proteolysis associated with antigen processing and presentation [GO:0002629] (biological process) Definition: Any process that stops, prevents, or reduces the frequency, rate, or extent of proteolysis associated with antigen processing and presentation. Sources: GOC:add Also known as: down regulation of proteolysis associated with antigen processing and presentation, down-regulation of proteolysis associated with antigen processing and presentation, downregulation of proteolysis associated with antigen processing and presentation, inhibition of proteolysis associated with antigen processing and presentation Relationships: is a type of negative regulation of antigen processing and presentation of peptide antigen [GO:0002584]; is a type of regulation of proteolysis associated with antigen processing and presentation [GO:0002628]; is_a negative regulation of protein catabolic process [GO:0042177]; is a type of negative regulation of proteolysis involved in protein catabolic process [GO:1903051]; negatively regulates proteolysis associated with antigen processing and presentation [GO:0002496]